{
  "gene_name": "ADAMTS-like protein 3",
  "gene": "UniProtKB:P82987",
  "term_label": "extracellular matrix",
  "gene_symbol": "ADAMTSL3",
  "term_id": "GO:0031012"
}